{
  "term_label": "Unknown cellular component",
  "gene": "UniProtKB:Q6T310",
  "term_id": "UNKNOWN:0003",
  "gene_symbol": "RASL11A",
  "gene_name": "Ras-like protein family member 11A"
}